protein localization to chloroplast [GO:0072598] (biological process) Subtypes: protein import into chloroplast stroma [GO:0045037], protein import into chloroplast thylakoid membrane [GO:0045038], protein localization to chloroplast starch grain [GO:1904160] Definition: A process in which a protein is transported to, or maintained at, a location in a chloroplast. Sources: GOC:ecd Relationships: is a type of protein localization to organelle [GO:0033365] Also known as: protein localisation to chloroplast